{
  "term_id": "GO:0007283",
  "gene_name": "BTB_POZ domain-containing protein 18",
  "term_label": "spermatogenesis",
  "gene": "UniProtKB:B2RXH4",
  "gene_symbol": "BTBD18"
}